{
  "gene_symbol": "REXO1L1P",
  "term_label": "exonuclease activity",
  "gene_name": "Putative exonuclease GOR",
  "term_id": "GO:0004527",
  "gene": "UniProtKB:Q8IX06"
}